{
  "gene_symbol": "KLHL1",
  "gene": "UniProtKB:Q9NR64",
  "term_id": "GO:0043025",
  "term_label": "neuronal cell body",
  "gene_name": "Kelch-like protein 1"
}